zona limitans intrathalamica formation [GO:0022006] (biological process) Also known as: zli biosynthesis, zli formation Relationships: is a type of formation of anatomical boundary [GO:0048859]; is part of rostrocaudal neural tube patterning [GO:0021903] References: PMID:11425897, PMID:16452095 Sources: GOC:cls, GOC:dgh, GOC:dph, GOC:jid, GO_REF:0000021 Definition: The formation of the narrow stripe of cells that lies between the prospective dorsal and ventral thalami. This boundary contains signals that pattern the prethalamic and thalamic territories of the future mid-diencephalon.